{
  "gene_symbol": "SYCE3",
  "gene": "UniProtKB:A1L190",
  "gene_name": "Synaptonemal complex central element protein 3",
  "term_label": "Unknown molecular function",
  "term_id": "UNKNOWN:0001"
}